polyamine deacetylation [GO:0106047] (biological process) Definition: The modification of acetylpolyamine by the removal of acetyl groups. References: PMID:28516954 Relationships: is a type of polyamine metabolic process [GO:0006595]; is a type of macromolecule deacylation [GO:0098732] Subtypes: spermidine deacetylation [GO:0106048]